{
  "gene_symbol": "SP9",
  "term_id": "GO:0000978",
  "gene_name": "Transcription factor Sp9",
  "gene": "UniProtKB:P0CG40",
  "term_label": "RNA polymerase II cis-regulatory region sequence-specific DNA binding"
}